{
  "term_id": "GO:0004112",
  "term_label": "cyclic-nucleotide phosphodiesterase activity",
  "gene_symbol": "MPPED2",
  "gene_name": "Metallophosphoesterase MPPED2",
  "gene": "UniProtKB:Q15777"
}